positive regulation of Fc receptor mediated stimulatory signaling pathway [GO:0060369] (biological process) Sources: GOC:BHF, GOC:dph, GOC:tb Subtypes: positive regulation of Fc-gamma receptor signaling pathway involved in phagocytosis [GO:1905451] Also known as: positive regulation of Fc receptor mediated stimulatory signalling pathway Definition: Any process that increases the rate, frequency or extent of the Fc receptor mediated stimulatory signaling pathway. Relationships: is a type of positive regulation of signal transduction [GO:0009967]; is a type of GO:0050778; is a type of GO:0060368; positively regulates Fc receptor mediated stimulatory signaling pathway [GO:0002431]